{
  "gene_name": "AP-1 complex subunit sigma-2",
  "gene_symbol": "AP1S2",
  "gene": "UniProtKB:P56377",
  "term_id": "UNKNOWN:0001",
  "term_label": "Unknown molecular function"
}